regulation of telomeric D-loop disassembly [GO:1905838] (biological process) Definition: Any process that modulates the frequency, rate or extent of telomeric D-loop disassembly. References: PMID:15200954 Sources: GOC:BHF, GOC:BHF_telomere, GOC:TermGenie, GOC:nc, GO_REF:0000058 Relationships: is a type of regulation of telomeric loop disassembly [GO:1904533]; regulates telomeric D-loop disassembly [GO:0061820] Subtypes: negative regulation of telomeric D-loop disassembly [GO:1905839], positive regulation of telomeric D-loop disassembly [GO:1905840]